{
  "gene": "UniProtKB:Q9Y6Q1",
  "term_id": "UNKNOWN:0002",
  "term_label": "Unknown biological process",
  "gene_symbol": "CAPN6",
  "gene_name": "Calpain-6"
}